O-hydroxycinnamoyltransferase activity [GO:0050737] (molecular function) Sources: GOC:ai Relationships: is a type of O-acyltransferase activity [GO:0008374]; is a type of GO:0050734 Subtypes: tartronate O-hydroxycinnamoyltransferase activity [GO:0047161], GO:0047169, glucarate O-hydroxycinnamoyltransferase activity [GO:0047170], glucarolactone O-hydroxycinnamoyltransferase activity [GO:0047171], GO:0047172, chlorogenate-glucarate O-hydroxycinnamoyltransferase activity [GO:0047204], quinate O-hydroxycinnamoyltransferase activity [GO:0047205] Definition: Catalysis of the transfer of a hydroxycinnamoyl group to an oxygen atom on the acceptor molecule.